{
  "term_label": "MHC class I protein complex binding",
  "term_id": "GO:0023024",
  "gene_symbol": "TAPBP",
  "gene_name": "Tapasin",
  "gene": "UniProtKB:O15533"
}